{
  "gene_symbol": "PIGN",
  "term_label": "GPI anchor biosynthetic process",
  "gene_name": "GPI ethanolamine phosphate transferase 1",
  "gene": "UniProtKB:O95427",
  "term_id": "GO:0006506"
}